{
  "gene_name": "Homeobox domain-containing protein",
  "term_id": "GO:0006357",
  "gene": "UniProtKB:A0A1B0GW55",
  "term_label": "regulation of transcription by RNA polymerase II",
  "gene_symbol": "LOC124905412"
}